{
  "term_id": "GO:0006357",
  "gene_name": "Zinc finger protein 844",
  "gene_symbol": "ZNF844",
  "gene": "UniProtKB:Q08AG5",
  "term_label": "regulation of transcription by RNA polymerase II"
}